glucuronosyl-N-acetylgalactosaminyl-proteoglycan 4-beta-N-acetylgalactosaminyltransferase activity [GO:0047238] (molecular function) Sources: EC:2.4.1.175 Relationships: is a type of GO:0008376 Definition: Catalysis of the reaction: D-glucuronyl-N-acetyl-1,3-beta-D-galactosaminylproteoglycan + UDP-N-acetylgalactosamine = N-acetyl-D-galactosaminyl-1,4-beta-D-glucuronyl-N-acetyl-1,3-beta-D-galactosaminylproteoglycan + UDP. Also known as: N-acetylgalactosaminyltransferase II activity, glucuronyl-N-acetylgalactosaminylproteoglycan 4-beta-N-acetylgalactosaminyltransferase activity, glucuronyl-N-acetylgalactosaminylproteoglycan beta-1,4-N-acetylgalactosaminyltransferase activity, UDP-N-acetyl-D-galactosamine:D-glucuronyl-N-acetyl-1,3-beta-D-galactosaminylproteoglycan beta-1,4-N-acetylgalactosaminyltransferase activity, UDP-N-acetyl-D-galactosamine:beta-D-glucuronosyl-(1->3)-N-acetyl-beta-D-galactosaminyl-proteoglycan 4-beta-N-acetylgalactosaminyltransferase activity, chondroitin synthase activity, uridine diphosphoacetylgalactosamine-chondroitin acetylgalactosaminyltransferase II activity